{
  "gene_symbol": "LBP",
  "gene_name": "Lipopolysaccharide-binding protein",
  "term_id": "GO:0043032",
  "term_label": "positive regulation of macrophage activation",
  "gene": "UniProtKB:P18428"
}